regulation of lipoprotein transport [GO:0140075] (biological process) References: PMID:26501192 Sources: GOC:BHF, GOC:BHF_miRNA, GOC:RPH Subtypes: negative regulation of lipoprotein transport [GO:0140076], positive regulation of lipoprotein transport [GO:0140077] Relationships: is a type of regulation of protein transport [GO:0051223]; RO_0002211 lipoprotein transport [GO:0042953] Definition: Any process that controls lipoprotein transport.